{
  "gene_symbol": "SENP3",
  "term_id": "GO:0016926",
  "gene_name": "Sentrin-specific protease 3",
  "term_label": "protein desumoylation",
  "gene": "UniProtKB:Q9H4L4"
}